vesicle cargo loading [GO:0035459] (biological process) Definition: The formation of a macromolecular complex between the coat proteins and proteins and/or lipoproteins that are going to be transported by a vesicle. Sources: GOC:bf, GOC:lb Also known as: cargo loading into vesicle, cargo selection Relationships: is a type of transport [GO:0006810]; is part of GO:0016192 Subtypes: clathrin-coated vesicle cargo loading [GO:0035652], COPII-coated vesicle cargo loading [GO:0090110]